{
  "gene_symbol": "DMPK",
  "gene": "UniProtKB:Q09013",
  "term_label": "regulation of heart contraction",
  "term_id": "GO:0008016",
  "gene_name": "Myotonin-protein kinase"
}